{
  "gene_symbol": "FFAR1",
  "term_label": "G protein-coupled receptor signaling pathway",
  "gene": "UniProtKB:O14842",
  "gene_name": "Free fatty acid receptor 1",
  "term_id": "GO:0007186"
}